{
  "gene_symbol": "CKS2",
  "gene": "UniProtKB:P33552",
  "term_label": "cyclin-dependent protein kinase holoenzyme complex",
  "term_id": "GO:0000307",
  "gene_name": "Cyclin-dependent kinases regulatory subunit 2"
}